{
  "term_label": "Unknown molecular function",
  "term_id": "UNKNOWN:0001",
  "gene": "UniProtKB:Q969S8",
  "gene_name": "Polyamine deacetylase HDAC10",
  "gene_symbol": "HDAC10"
}